{
  "gene": "UniProtKB:Q8IWL8",
  "term_id": "UNKNOWN:0002",
  "term_label": "Unknown biological process",
  "gene_symbol": "STH",
  "gene_name": "Saitohin"
}